{
  "gene_symbol": "EPB41L4A",
  "term_label": "Unknown molecular function",
  "gene": "UniProtKB:Q9HCS5",
  "term_id": "UNKNOWN:0001",
  "gene_name": "Band 4.1-like protein 4A"
}